{
  "term_label": "positive regulation of cold-induced thermogenesis",
  "term_id": "GO:0120162",
  "gene_name": "Mitochondrial brown fat uncoupling protein 1",
  "gene_symbol": "UCP1",
  "gene": "UniProtKB:P25874"
}